{
  "term_label": "inositol phosphate biosynthetic process",
  "gene_name": "Inositol hexakisphosphate kinase 3",
  "gene": "UniProtKB:Q96PC2",
  "gene_symbol": "IP6K3",
  "term_id": "GO:0032958"
}